{
  "gene": "UniProtKB:F8WBI6",
  "term_id": "GO:0007030",
  "gene_symbol": "GOLGA8N",
  "gene_name": "Golgin subfamily A member 8N",
  "term_label": "Golgi organization"
}